{
  "gene_symbol": "FTO",
  "gene": "UniProtKB:Q9C0B1",
  "gene_name": "Alpha-ketoglutarate-dependent dioxygenase FTO",
  "term_label": "regulation of lipid storage",
  "term_id": "GO:0010883"
}